corticosteroid side-chain-isomerase activity [GO:0004110] (molecular function) Sources: EC:5.3.1.21, RHEA:17861 Also known as: 11-deoxycorticosterone aldose-ketose-isomerase activity, 11-deoxycorticosterone ketol-isomerase activity Definition: Catalysis of the reaction: 11-deoxycorticosterone = 20-hydroxy-3-oxopregn-4-en-21-al. Relationships: is a type of intramolecular oxidoreductase activity, interconverting aldoses and ketoses [GO:0016861]